protein to membrane docking [GO:0022615] (biological process) Definition: The initial attachment of a protein to a target membrane, mediated by a proteins protruding from the target membrane. Docking requires only that the proteins come close enough to interact and adhere. Sources: GOC:isa_complete Subtypes: GO:0006615 Also known as: protein-membrane docking Relationships: is a type of membrane docking [GO:0022406]